ubiquitin conjugating enzyme activity [GO:0061631] (molecular function) Sources: GOC:BioGRID, GOC:dph Definition: Isoenergetic transfer of ubiquitin from one protein to another via the reaction X-ubiquitin + Y = Y-ubiquitin + X, where both the X-ubiquitin and Y-ubiquitin linkages are thioester bonds between the C-terminal glycine of ubiquitin and a sulfhydryl side group of a cysteine residue. Also known as: E2, HECT E3 Relationships: is a type of GO:0004842; is a type of ubiquitin-like protein conjugating enzyme activity [GO:0061650]